toluene-4-sulfonate catabolic process [GO:0046269] (biological process) Definition: The chemical reactions and pathways resulting in the breakdown of toluene-4-sulfonate, 4-methylbenzenesulfonate, the anion of sulfonic acid attached to a methylbenzene molecule. Also known as: 4-toluenesulfonate catabolic process, 4-toluenesulfonate catabolism, toluene-4-sulfonate breakdown, toluene-4-sulfonate catabolism, toluene-4-sulfonate degradation, toluene-4-sulphonate catabolic process, toluene-4-sulphonate catabolism Sources: GOC:ai Relationships: is a type of GO:0016054; is a type of GO:0044273; is_a toluene-containing compound catabolic process [GO:0072491]